phycocyanobilin:ferredoxin oxidoreductase activity [GO:0050620] (molecular function) Definition: Catalysis of the reaction: (3Z)-phycocyanobilin + oxidized ferredoxin = biliverdin IXa + reduced ferredoxin. Also known as: (3Z)-phycocyanobilin:ferredoxin oxidoreductase activity Relationships: is a type of GO:0016636 Sources: EC:1.3.7.5, MetaCyc:1.3.7.5-RXN